{
  "gene_name": "PRKCA-binding protein",
  "term_id": "GO:0034315",
  "gene": "UniProtKB:Q9NRD5",
  "gene_symbol": "PICK1",
  "term_label": "regulation of Arp2/3 complex-mediated actin nucleation"
}